amyloplast ADPG pyrophosphorylase complex [GO:0030932] (cellular component) Relationships: is a type of plastid ADPG pyrophosphorylase complex [GO:0031009]; is part of amyloplast [GO:0009501] Definition: An ADPG pyrophosphorylase complex found in the amyloplast. Sources: GOC:mah